{
  "gene_name": "General transcription factor IIH subunit 1",
  "term_label": "transcription by RNA polymerase II",
  "gene_symbol": "GTF2H1",
  "gene": "UniProtKB:P32780",
  "term_id": "GO:0006366"
}